{
  "gene_symbol": "MARK4",
  "term_label": "intracellular signal transduction",
  "term_id": "GO:0035556",
  "gene_name": "MAP_microtubule affinity-regulating kinase 4",
  "gene": "UniProtKB:Q96L34"
}